{
  "gene_symbol": "PPARG",
  "term_label": "RNA polymerase II cis-regulatory region sequence-specific DNA binding",
  "gene_name": "Peroxisome proliferator-activated receptor gamma",
  "term_id": "GO:0000978",
  "gene": "UniProtKB:P37231"
}